{
  "gene_symbol": "SLC35E2A",
  "gene": "UniProtKB:P0CK97",
  "term_id": "GO:0015297",
  "term_label": "antiporter activity",
  "gene_name": "Solute carrier family 35 member E2A"
}